{
  "gene": "UniProtKB:O75690",
  "term_label": "Unknown molecular function",
  "gene_symbol": "KRTAP5-8",
  "term_id": "UNKNOWN:0001",
  "gene_name": "Keratin-associated protein 5-8"
}